{
  "gene_symbol": "CATSPERB",
  "gene_name": "Cation channel sperm-associated auxiliary subunit beta",
  "term_label": "Unknown biological process",
  "term_id": "UNKNOWN:0002",
  "gene": "UniProtKB:Q9H7T0"
}